trachea cartilage development [GO:0060534] (biological process) Definition: The process whose specific outcome is the progression of the tracheal cartilage over time, from its formation to the mature structure. Cartilage is a connective tissue dominated by extracellular matrix containing collagen type II and large amounts of proteoglycan, particularly chondroitin sulfate. Sources: GOC:dph Relationships: is a type of GO:0051216; BFO_0000050 trachea development [GO:0060438]